{
  "gene_symbol": "CFB",
  "gene_name": "Complement factor B",
  "term_id": "UNKNOWN:0001",
  "gene": "UniProtKB:P00751",
  "term_label": "Unknown molecular function"
}